{
  "gene_name": "Membrane-associated phosphatidylinositol transfer protein 3",
  "gene": "UniProtKB:Q9BZ71",
  "term_id": "GO:0004620",
  "gene_symbol": "PITPNM3",
  "term_label": "phospholipase activity"
}